host-mediated perturbation of viral process [GO:0044788] (biological process) Relationships: is_a host-mediated perturbation of symbiont process [GO:0051851] Definition: A process in which a host organism alters or subverts a biological process being mediated by a virus with which it is infected. Subtypes: host-mediated perturbation of viral transcription [GO:0043921], host-mediated suppression of viral proces [GO:0044793], host-mediated activation of viral process [GO:0044794], GO:0044827, host-mediated suppression of viral genome replication [GO:0044828], host-mediated perturbation of viral RNA genome replication [GO:0044830], modulation by host of viral molecular function [GO:0044868], modulation by host of viral glycoprotein metabolic process [GO:0044870] Also known as: modulation by host of viral process Sources: GOC:jl